{
  "term_id": "UNKNOWN:0003",
  "gene_name": "T cell receptor beta diversity 1",
  "gene": "UniProtKB:P0DPI4",
  "term_label": "Unknown cellular component",
  "gene_symbol": "TRBD1"
}